{
  "gene_name": "Store-operated calcium entry-associated regulatory factor",
  "gene_symbol": "SARAF",
  "term_label": "Unknown molecular function",
  "gene": "UniProtKB:Q96BY9",
  "term_id": "UNKNOWN:0001"
}